{
  "gene_name": "Solute carrier family 2, facilitated glucose transporter member 9",
  "gene": "UniProtKB:Q9NRM0",
  "gene_symbol": "SLC2A9",
  "term_id": "GO:0070837",
  "term_label": "dehydroascorbic acid transport"
}